histone H3K36me3 reader activity [GO:0140003] (molecular function) References: PMID:15489290, PMID:16364921 Relationships: is a type of GO:0140006 Definition: A histone reader that recognizes a histone H3 trimethylated at lysine 36. Note: Comment: Note that the residue position corresponds to the canonical human H3 histone (UniProtKB:P84243); this residue is conserved across all eukaryotes. Residue 1 is the first residue following removal of the initiating Methionine (Met). Note that each histone is encoded by multiple genes, and sequences may vary across different genes within an organism. Also known as: H3-K36me3 modified histone binding, H3K36me3 modified histone binding